{
  "gene": "UniProtKB:Q06141",
  "gene_symbol": "REG3A",
  "gene_name": "Regenerating islet-derived protein 3-alpha",
  "term_label": "response to peptide hormone",
  "term_id": "GO:0043434"
}